{
  "gene_name": "PDZ and LIM domain protein 2",
  "gene_symbol": "PDLIM2",
  "term_label": "muscle alpha-actinin binding",
  "term_id": "GO:0051371",
  "gene": "UniProtKB:Q96JY6"
}